{
  "term_label": "Unknown molecular function",
  "gene_name": "Ubiquitin carboxyl-terminal hydrolase 4",
  "gene_symbol": "USP4",
  "gene": "UniProtKB:Q13107",
  "term_id": "UNKNOWN:0001"
}